{
  "gene": "UniProtKB:Q8N6Y1",
  "term_label": "plasma membrane",
  "gene_symbol": "PCDH20",
  "term_id": "GO:0005886",
  "gene_name": "Protocadherin-20"
}